asexual reproduction [GO:0019954] (biological process) Also known as: parthenogenesis References: PMID:22977071, PMID:28779329, PMID:29559496 Sources: ISBN:0387520546 Subtypes: cell budding [GO:0007114], asexual sporulation [GO:0030436], plantlet formation on parent plant [GO:0048624] Regulation: regulated by regulation of asexual reproduction [GO:1903664]; negatively regulated by negative regulation of asexual reproduction [GO:1903665]; positively regulated by positive regulation of asexual reproduction [GO:1903666] Definition: A type of reproduction in which new individuals are produced from a single organism, either from an unfertilized egg or from a single cell or group of cells. Relationships: is a type of reproductive process [GO:0022414]